{
  "term_id": "GO:0006508",
  "term_label": "proteolysis",
  "gene_name": "Prolactin-inducible protein",
  "gene": "UniProtKB:P12273",
  "gene_symbol": "PIP"
}